{
  "gene_symbol": "CSF1R",
  "term_label": "macrophage colony-stimulating factor receptor activity",
  "gene_name": "Macrophage colony-stimulating factor 1 receptor",
  "gene": "UniProtKB:P07333",
  "term_id": "GO:0005011"
}